purine nucleoside catabolic process [GO:0006152] (biological process) Definition: The chemical reactions and pathways resulting in the breakdown of purine nucleoside, one of a family of organic molecules consisting of a purine base covalently bonded to a sugar ribose (a ribonucleoside) or deoxyribose (a deoxyribonucleoside). Sources: GOC:go_curators Also known as: purine nucleoside breakdown, purine nucleoside catabolism, purine nucleoside degradation Relationships: is a type of GO:0009164; is a type of purine nucleoside metabolic process [GO:0042278]; is a type of purine-containing compound catabolic process [GO:0072523] Subtypes: purine deoxyribonucleoside catabolic process [GO:0046124], GO:0046130